glyoxalase (glycolic acid-forming) activity [GO:1990422] (molecular function) References: PMID:22523093 Sources: GOC:PARL, GOC:bf Relationships: is a type of hydro-lyase activity [GO:0016836]; is part of glycolate biosynthetic process [GO:0046295]; is part of GO:1903190 Definition: Catalysis of the reaction: glyoxal + H2O = glycolic acid. Catalysis occurs in the absence of a cofactor.